{
  "term_id": "GO:0031468",
  "gene_symbol": "CHMP7",
  "gene_name": "Charged multivesicular body protein 7",
  "term_label": "nuclear membrane reassembly",
  "gene": "UniProtKB:Q8WUX9"
}